{
  "gene_name": "SUN domain-containing protein 3",
  "term_id": "UNKNOWN:0002",
  "term_label": "Unknown biological process",
  "gene": "UniProtKB:Q8TAQ9",
  "gene_symbol": "SUN3"
}